{
  "gene_name": "ADP-ribosylation factor-like protein 11",
  "term_id": "GO:0006886",
  "gene": "UniProtKB:Q969Q4",
  "term_label": "intracellular protein transport",
  "gene_symbol": "ARL11"
}